{
  "term_label": "Unknown biological process",
  "gene_symbol": "CIMAP1A",
  "gene": "UniProtKB:Q96PU9",
  "term_id": "UNKNOWN:0002",
  "gene_name": "Outer dense fiber protein 3"
}